isoflavone 2'-hydroxylase activity [GO:0033773] (molecular function) Relationships: is a type of oxidoreductase activity, acting on paired donors, with incorporation or reduction of molecular oxygen, reduced flavin or flavoprotein as one donor, and incorporation of one atom of oxygen [GO:0016712] Definition: Catalysis of the reaction: an isoflavone + O2 + reduced [NADPH-hemoprotein reductase] = a 2'-hydroxyisoflavone + H+ + H2O + oxidized [NADPH-hemoprotein reductase]. Also known as: isoflavone 2'-monooxygenase activity, CYP Ge-3, CYP81E1 Sources: RHEA:18849